{
  "term_id": "UNKNOWN:0001",
  "gene_symbol": "CABLES1",
  "gene_name": "CDK5 and ABL1 enzyme substrate 1",
  "gene": "UniProtKB:Q8TDN4",
  "term_label": "Unknown molecular function"
}